{
  "term_id": "UNKNOWN:0001",
  "term_label": "Unknown molecular function",
  "gene_symbol": "DUOXA1",
  "gene_name": "Dual oxidase maturation factor 1",
  "gene": "UniProtKB:Q1HG43"
}